venom-mediated smooth muscle relaxation [GO:0044617] (biological process) Also known as: modulation of relaxation of smooth muscle in other organism, regulation of relaxation of smooth muscle in other organism, modulation of relaxation of smooth muscle in another organism Definition: A process in which an organism initiates, promotes, or enhances the relaxation of smooth muscle in another organism via the action of a venom. Sources: GOC:jl Relationships: is a type of GO:0140137